{
  "gene_symbol": "EIF4ENIF1",
  "gene_name": "Eukaryotic translation initiation factor 4E transporter",
  "gene": "UniProtKB:Q9NRA8",
  "term_id": "GO:0003729",
  "term_label": "mRNA binding"
}